{
  "term_label": "plasma membrane",
  "gene_symbol": "ADCYAP1R1",
  "gene": "UniProtKB:P41586",
  "term_id": "GO:0005886",
  "gene_name": "Pituitary adenylate cyclase-activating polypeptide type I receptor"
}